{
  "gene": "UniProtKB:P0DMU8",
  "gene_name": "Cancer_testis antigen family 45 member A5",
  "term_id": "UNKNOWN:0002",
  "gene_symbol": "CT45A5",
  "term_label": "Unknown biological process"
}